{
  "term_id": "UNKNOWN:0003",
  "gene_name": "Alanine and arginine-rich domain-containing protein",
  "gene": "UniProtKB:Q4LEZ3",
  "term_label": "Unknown cellular component",
  "gene_symbol": "AARD"
}